{
  "term_id": "GO:0007043",
  "gene": "UniProtKB:P55290",
  "gene_name": "Cadherin-13",
  "term_label": "cell-cell junction assembly",
  "gene_symbol": "CDH13"
}